{
  "gene_symbol": "GCSH",
  "gene_name": "Glycine cleavage system H protein, mitochondrial",
  "gene": "UniProtKB:P23434",
  "term_label": "glycine decarboxylation via glycine cleavage system",
  "term_id": "GO:0019464"
}